{
  "gene_name": "Putative HIG1 domain family member 2B",
  "gene_symbol": "HIGD2B",
  "term_label": "mitochondrion",
  "term_id": "GO:0005739",
  "gene": "UniProtKB:Q4VC39"
}